positive regulation of transcription by transcription factor localization [GO:0061586] (biological process) Relationships: is a type of intracellular protein localization [GO:0008104]; is a type of positive regulation of DNA-templated transcription [GO:0045893] Sources: GOC:dph Definition: Any process that activates or increases the frequency, rate or extent of DNA-dependent transcription using a mechanism that involves the localization of a transcription factor.